{
  "term_label": "Unknown cellular component",
  "gene_symbol": "SS18L2",
  "term_id": "UNKNOWN:0003",
  "gene_name": "SS18-like protein 2",
  "gene": "UniProtKB:Q9UHA2"
}